{
  "gene_name": "Oxysterol-binding protein-related protein 9",
  "gene": "UniProtKB:Q96SU4",
  "term_id": "GO:0005794",
  "gene_symbol": "OSBPL9",
  "term_label": "Golgi apparatus"
}